{
  "term_id": "GO:0015193",
  "gene": "UniProtKB:Q9NP91",
  "gene_name": "Sodium- and chloride-dependent transporter XTRP3",
  "gene_symbol": "SLC6A20",
  "term_label": "L-proline transmembrane transporter activity"
}